{
  "term_label": "cell surface",
  "term_id": "GO:0009986",
  "gene_name": "Junctional adhesion molecule B",
  "gene_symbol": "JAM2",
  "gene": "UniProtKB:P57087"
}